{
  "gene_name": "Frizzled-5",
  "term_label": "plasma membrane",
  "term_id": "GO:0005886",
  "gene_symbol": "FZD5",
  "gene": "UniProtKB:Q13467"
}